{
  "term_id": "GO:0005615",
  "term_label": "extracellular space",
  "gene_symbol": "DEFA1B",
  "gene_name": "Neutrophil defensin 1",
  "gene": "UniProtKB:P59665"
}